{
  "gene": "UniProtKB:O95905",
  "term_id": "UNKNOWN:0001",
  "term_label": "Unknown molecular function",
  "gene_name": "Protein ecdysoneless homolog",
  "gene_symbol": "ECD"
}